{
  "gene": "UniProtKB:O95661",
  "term_id": "GO:0003924",
  "term_label": "GTPase activity",
  "gene_name": "GTP-binding protein Di-Ras3",
  "gene_symbol": "DIRAS3"
}